{
  "gene_name": "N-acyl-phosphatidylethanolamine-hydrolyzing phospholipase D",
  "term_id": "GO:0043025",
  "term_label": "neuronal cell body",
  "gene_symbol": "NAPEPLD",
  "gene": "UniProtKB:Q6IQ20"
}